{
  "gene_symbol": "CTAGE1",
  "gene": "UniProtKB:Q96RT6",
  "term_id": "GO:0035459",
  "term_label": "vesicle cargo loading",
  "gene_name": "cTAGE family member 2"
}